MAML2-RBP-Jkappa-ICN1 complex [GO:0071175] (CC) Also known as: MAML2-RBP-Jkappa-Notch1 complex References: PMID:12370315 Relationships: is a type of nuclear protein-containing complex [GO:0140513] Definition: A protein complex that consists of the intracellular domain of Notch1 (ICN1), the DNA-binding transcription factor RBP-Jkappa, and the transcriptional coactivator Mastermind-like-2 (MAML2); the complex is involved in transcriptional activation in response to Notch-mediated signaling.